indole alkaloid biosynthetic process [GO:0035835] (biological process) Subtypes: GO:0009709, psilocybin biosynthetic process [GO:0140380], tryprostatin A biosynthetic process [GO:0140654], GO:1900772, fumiquinazoline C biosynthetic process [GO:1900781], brevianamide F biosynthetic process [GO:1900805], 3alpha(S)-strictosidine biosynthetic process [GO:1901015], verruculogen biosynthetic process [GO:1902181] Sources: GOC:yaf Also known as: indole alkaloid anabolism, indole alkaloid biosynthesis, indole alkaloid formation, indole alkaloid synthesis Definition: The chemical reactions and pathways resulting in the formation of an indole alkaloid, an alkaloid containing an indole skeleton. Relationships: is_a alkaloid biosynthetic process [GO:0009821]; is a type of indole alkaloid metabolic process [GO:0035834]